{
  "term_id": "UNKNOWN:0003",
  "term_label": "Unknown cellular component",
  "gene": "UniProtKB:Q9NS85",
  "gene_symbol": "CA10",
  "gene_name": "Carbonic anhydrase-related protein 10"
}